alkanesulfonate catabolic process [GO:0046306] (biological process) Sources: GOC:ai Subtypes: GO:0019529 Relationships: is a type of organic acid catabolic process [GO:0016054]; is_a alkanesulfonate metabolic process [GO:0019694]; is a type of sulfur compound catabolic process [GO:0044273] Also known as: alkanesulfonate breakdown, alkanesulfonate catabolism, alkanesulfonate degradation, alkanesulphonate catabolic process, alkanesulphonate catabolism Definition: The chemical reactions and pathways resulting in the breakdown of alkanesulfonates, the anion of alkanesulfonic acids, sulfonic acid derivatives containing an aliphatic hydrocarbon group.